{
  "term_id": "GO:0000398",
  "gene": "UniProtKB:P98179",
  "term_label": "mRNA splicing, via spliceosome",
  "gene_name": "RNA-binding protein 3",
  "gene_symbol": "RBM3"
}